{
  "term_id": "UNKNOWN:0001",
  "gene_name": "Palmitoyltransferase ZDHHC17",
  "term_label": "Unknown molecular function",
  "gene": "UniProtKB:Q8IUH5",
  "gene_symbol": "ZDHHC17"
}